cell wall polysaccharide catabolic process involved in abscission [GO:1990076] (biological process) References: PMID:23479623 Sources: GOC:TermGenie Definition: Any cell wall polysaccharide catabolic process that is involved in abscission. Relationships: is a type of cell wall polysaccharide catabolic process [GO:0044347]; BFO_0000050 GO:0009838